{
  "term_id": "UNKNOWN:0001",
  "gene_name": "Cytochrome b-245 light chain",
  "gene_symbol": "CYBA",
  "gene": "UniProtKB:P13498",
  "term_label": "Unknown molecular function"
}